{
  "term_id": "GO:0005886",
  "gene_symbol": "TACR1",
  "gene_name": "Substance-P receptor",
  "gene": "UniProtKB:P25103",
  "term_label": "plasma membrane"
}